serotonin catabolic process [GO:0042429] (biological process) Sources: GOC:jl, ISBN:0198506732 Also known as: serotonin breakdown, serotonin catabolism, serotonin degradation Definition: The chemical reactions and pathways resulting in the breakdown of serotonin (5-hydroxytryptamine), a monoamine neurotransmitter occurring in the peripheral and central nervous systems, also having hormonal properties. Relationships: is a type of phenol-containing compound catabolic process [GO:0019336]; is a type of GO:0042428; is a type of GO:0042436; is a type of primary amino compound catabolic process [GO:1901161]